protein heterotrimerization [GO:0070208] (biological process) Definition: The formation of a protein heterotrimer, a macromolecular structure consisting of three noncovalently associated subunits, of which not all are identical. Also known as: protein heterotrimer assembly, protein heterotrimer biosynthesis, protein heterotrimer biosynthetic process, protein heterotrimer formation Sources: GOC:hjd Relationships: is a type of protein heterooligomerization [GO:0051291]; is a type of protein trimerization [GO:0070206]